acyl binding [GO:0000035] (molecular function) Also known as: acyl-CoA or acyl binding Definition: Binding to an acyl group, any group formally derived by removal of the hydroxyl group from the acid function of a carboxylic acid. Relationships: is a type of small molecule binding [GO:0036094] Sources: GOC:curators, ISBN:0198506732